septate junction [GO:0005918] (cellular component) Relationships: is a type of GO:0070160; is part of GO:0043296 Also known as: septate desmosome References: PMID:11700298, PMID:12612641, PMID:20795303, PMID:28636800 Sources: ISBN:0815332181 Definition: A cell-cell junction that forms a continuous band around each cell in an epithelium; within the septate junction the membranes of adjacent cells maintain a constant distance of approximately 15 nm; found in arthropods. Subtypes: GO:0005919, smooth septate junction [GO:0005920]